{
  "gene": "UniProtKB:Q8NGY0",
  "term_label": "Unknown molecular function",
  "term_id": "UNKNOWN:0001",
  "gene_name": "Olfactory receptor 10X1",
  "gene_symbol": "OR10X1"
}